{
  "gene_name": "Protein kish-A",
  "gene_symbol": "TMEM167A",
  "term_label": "protein secretion",
  "gene": "UniProtKB:Q8TBQ9",
  "term_id": "GO:0009306"
}